{
  "term_label": "phosphatidylinositol binding",
  "gene": "UniProtKB:Q9Y5X1",
  "term_id": "GO:0035091",
  "gene_name": "Sorting nexin-9",
  "gene_symbol": "SNX9"
}